{
  "term_id": "GO:0031430",
  "term_label": "M band",
  "gene_symbol": "MYOM1",
  "gene": "UniProtKB:P52179",
  "gene_name": "Myomesin-1"
}